{
  "term_label": "tRNA (N(6)-L-threonylcarbamoyladenosine(37)-C(2))-methylthiotransferase activity",
  "term_id": "GO:0035598",
  "gene_symbol": "CDKAL1",
  "gene": "UniProtKB:Q5VV42",
  "gene_name": "Threonylcarbamoyladenosine tRNA methylthiotransferase"
}